androst-4-ene-3,17-dione biosynthetic process [GO:1903449] (biological process) Relationships: is_a steroid biosynthetic process [GO:0006694]; is a type of ketone biosynthetic process [GO:0042181]; is a type of olefinic compound biosynthetic process [GO:0120255] Also known as: androst-4-ene-3,17-dione anabolism, androst-4-ene-3,17-dione biosynthesis, androst-4-ene-3,17-dione formation, androst-4-ene-3,17-dione synthesis, androstenedione biosynthetic process References: PMID:2028480, PMID:4149619 Sources: GOC:TermGenie, GOC:mr, GO_REF:0000068 Definition: The chemical reactions and pathways resulting in the formation of androst-4-ene-3,17-dione. Regulation: regulated by regulation of androst-4-ene-3,17-dione biosynthetic process [GO:1903454]; negatively regulated by negative regulation of androst-4-ene-3,17-dione biosynthetic process [GO:1903455]; positively regulated by positive regulation of androst-4-ene-3,17-dione biosynthetic process [GO:1903456]